{
  "gene_symbol": "RTN1",
  "term_label": "endoplasmic reticulum tubular network membrane organization",
  "gene_name": "Reticulon-1",
  "gene": "UniProtKB:Q16799",
  "term_id": "GO:1990809"
}